{
  "gene_name": "Centrosomal protein of 19 kDa",
  "gene": "UniProtKB:Q96LK0",
  "term_id": "UNKNOWN:0001",
  "term_label": "Unknown molecular function",
  "gene_symbol": "CEP19"
}